ciliary basal body segregation [GO:0120312] (biological process) Relationships: is a type of cellular process [GO:0009987] Also known as: microtubule basal body segregation, ciliary basal body separation, microtubule basal body separation References: PMID:1876188, PMID:26272611, PMID:26862392, PMID:27252853, PMID:4055898 Sources: GOC:ach, GOC:krc Definition: The process in which the duplicated basal bodies migrate in pairs to the mitotic poles of the nucleus and results in equal distribution in the daughter cells. Ciliary basal body segregation ensures inheritance of the duplicated mitochondrial DNA to the two daughter cells in the Trypanosoma parasites.